mesenchyme morphogenesis [GO:0072132] (biological process) Sources: GOC:mtg_kidney_jan10 Subtypes: GO:0003203, paraxial mesoderm morphogenesis [GO:0048340], lateral mesoderm morphogenesis [GO:0048369], kidney mesenchyme morphogenesis [GO:0072131] Definition: The process in which the anatomical structures of a mesenchymal tissue are generated and organized. A mesenchymal tissue is made up of loosely packed stellate cells. Relationships: is a type of tissue morphogenesis [GO:0048729]; is part of animal organ morphogenesis [GO:0009887]; BFO_0000050 mesenchyme development [GO:0060485]